{
  "gene": "UniProtKB:Q9H3Z7",
  "gene_symbol": "ABHD16B",
  "term_label": "phospholipase activity",
  "term_id": "GO:0004620",
  "gene_name": "Protein ABHD16B"
}